filamentous growth of a population of unicellular organisms in response to heat [GO:0036168] (biological process) Relationships: is a type of response to heat [GO:0009408]; is a type of filamentous growth of a population of unicellular organisms [GO:0044182] References: PMID:17554048 Sources: GOC:di Definition: The process in which a group of unicellular organisms grow in a threadlike, filamentous shape in response to an increase in temperature. Subtypes: GO:0036165 Regulation: regulated by GO:1900431; negatively regulated by negative regulation of filamentous growth of a population of unicellular organisms in response to heat [GO:1900432]; RO_0002213 by GO:1900433